crystal cell differentiation [GO:0042688] (biological process) Sources: GOC:bf, http://sdb.bio.purdue.edu/fly/gene/serpent3.htm Subtypes: embryonic crystal cell differentiation [GO:0035165], lymph gland crystal cell differentiation [GO:0035170] Definition: The process in which a hemocyte precursor cell acquires the characteristics of a crystal cell, a class of cells that contain crystalline inclusions and are involved in the melanization of pathogenic material in the hemolymph. Regulation: regulated by regulation of crystal cell differentiation [GO:0042689]; negatively regulated by negative regulation of crystal cell differentiation [GO:0042690]; positively regulated by GO:0042691 Relationships: is a type of hemocyte differentiation [GO:0042386]